{
  "term_label": "integrin alpha2-beta1 complex",
  "gene_symbol": "ITGA2",
  "gene": "UniProtKB:P17301",
  "term_id": "GO:0034666",
  "gene_name": "Integrin alpha-2"
}